{
  "gene_name": "Membrane-associated phosphatidylinositol transfer protein 3",
  "gene": "UniProtKB:Q9BZ71",
  "term_label": "cytoplasm",
  "gene_symbol": "PITPNM3",
  "term_id": "GO:0005737"
}